negative regulation of isoprenoid metabolic process [GO:0045827] (biological process) Subtypes: negative regulation of isopentenyl diphosphate biosynthetic process, methylerythritol 4-phosphate pathway [GO:0010323], GO:0010373, negative regulation of juvenile hormone metabolic process [GO:0045928], negative regulation of abscisic acid biosynthetic process [GO:0090359], negative regulation of retinoic acid biosynthetic process [GO:1900053], GO:1900948, negative regulation of ent-pimara-8(14),15-diene biosynthetic process [GO:1901543], negative regulation of carotenoid biosynthetic process [GO:1904142], GO:2001211 Definition: Any process that stops, prevents, or reduces the frequency, rate or extent of the chemical reactions and pathways involving isoprenoid. Sources: GOC:go_curators Also known as: down regulation of isoprenoid metabolic process, down-regulation of isoprenoid metabolic process, downregulation of isoprenoid metabolic process, negative regulation of isoprenoid metabolism, inhibition of isoprenoid metabolic process Relationships: is a type of GO:0019747; is a type of negative regulation of lipid metabolic process [GO:0045833]; negatively regulates isoprenoid metabolic process [GO:0006720]